{
  "term_label": "myosin II complex",
  "gene": "UniProtKB:P14649",
  "term_id": "GO:0016460",
  "gene_name": "Myosin light chain 6B",
  "gene_symbol": "MYL6B"
}